{
  "term_label": "nuclear receptor-mediated steroid hormone signaling pathway",
  "gene_name": "G-protein coupled estrogen receptor 1",
  "gene_symbol": "GPER1",
  "term_id": "GO:0030518",
  "gene": "UniProtKB:Q99527"
}